{
  "gene_name": "Platelet-derived growth factor receptor alpha",
  "term_id": "GO:0005018",
  "gene_symbol": "PDGFRA",
  "term_label": "platelet-derived growth factor alpha-receptor activity",
  "gene": "UniProtKB:P16234"
}